{
  "gene_name": "Fibroblast growth factor receptor substrate 3",
  "gene_symbol": "FRS3",
  "gene": "UniProtKB:O43559",
  "term_label": "Unknown cellular component",
  "term_id": "UNKNOWN:0003"
}